synapse pruning [GO:0098883] (biological process) Subtypes: GO:0150062, excitatory synapse pruning [GO:1905805] Definition: A cellular process that results in the controlled breakdown of synapse. After it starts the process is continuous until the synapse has disappeared. References: PMID:12062020, PMID:18083105, PMID:22632716, PMID:29844190 Sources: GOC:dos Relationships: is a type of GO:0050808; is a type of cell junction disassembly [GO:0150146] Also known as: synapse clearance, synapse disassembly, synapse elimination, synapse removal Regulation: regulated by GO:1905806; negatively regulated by negative regulation of synapse pruning [GO:1905807]; positively regulated by positive regulation of synapse pruning [GO:1905808]